{
  "gene_symbol": "MOGS",
  "term_id": "GO:0004573",
  "gene": "UniProtKB:Q13724",
  "gene_name": "Mannosyl-oligosaccharide glucosidase",
  "term_label": "Glc3Man9GlcNAc2 oligosaccharide glucosidase activity"
}